{
  "term_label": "Unknown molecular function",
  "gene": "UniProtKB:Q8IXR5",
  "gene_name": "Protein FAM178B",
  "term_id": "UNKNOWN:0001",
  "gene_symbol": "FAM178B"
}